{
  "term_id": "GO:0030527",
  "gene": "UniProtKB:Q96QV6",
  "term_label": "structural constituent of chromatin",
  "gene_name": "Histone H2A type 1-A",
  "gene_symbol": "H2AC1"
}